{
  "gene_symbol": "ZMYM1",
  "gene": "UniProtKB:Q5SVZ6",
  "term_label": "Unknown biological process",
  "gene_name": "Zinc finger MYM-type protein 1",
  "term_id": "UNKNOWN:0002"
}